{
  "term_id": "GO:0005886",
  "gene_name": "Leukocyte surface antigen CD53",
  "gene_symbol": "CD53",
  "gene": "UniProtKB:P19397",
  "term_label": "plasma membrane"
}